presynaptic cytoskeleton [GO:0099569] (cellular component) Definition: The portion of the cytoskeleton contained within the presynapse. Sources: GOC:dos Relationships: is a type of cytoskeleton [GO:0005856]; is part of presynapse [GO:0098793] Subtypes: cytoskeleton of presynaptic active zone [GO:0048788], presynaptic actin cytoskeleton [GO:0099143], presynaptic intermediate filament cytoskeleton [GO:0099182]